serotonin receptor signaling pathway [GO:0007210] (biological process) Also known as: serotonin receptor signalling pathway Sources: GOC:mah Relationships: is a type of signal transduction [GO:0007165]; is part of cellular response to dopamine [GO:1903351]; has part serotonin receptor activity [GO:0099589] Subtypes: GO:0007192, serotonin-gated cation-selective signaling pathway [GO:0140227], positive regulation of fatty acid beta-oxidation by serotonin receptor signaling pathway [GO:1904123] Definition: The series of molecular signals generated as a consequence of a serotonin receptor binding to one of its physiological ligands.